fatty acid elongase activity [GO:0009922] (MF) Also known as: condensing enzyme, ELOVL, elongation of very long chain fatty acids activity, very-long-chain 3-ketoacyl-CoA synthase, very-long-chain 3-oxoacyl-CoA synthase, very-long-chain beta-ketoacyl-CoA synthase Relationships: is a type of acyltransferase activity, transferring groups other than amino-acyl groups [GO:0016747] References: PMID:16564093, PMID:19763486 Sources: RHEA:32727 Definition: Catalysis of the reaction: a very-long-chain acyl-CoA + H+ + malonyl-CoA = a very-long-chain 3-oxoacyl-CoA + CO2 + CoA. This reaction is the first (condensation) step of the four-step fatty acid elongation cycle in the endoplasmic reticulum that extends fatty acids of C-16 or longer with an additional 2-C unit.